{
  "gene": "UniProtKB:P20853",
  "term_label": "arachidonate epoxygenase activity",
  "gene_symbol": "CYP2A7",
  "gene_name": "Cytochrome P450 2A7",
  "term_id": "GO:0008392"
}